{
  "term_id": "GO:0005739",
  "gene_symbol": "PDPR",
  "gene": "UniProtKB:Q8NCN5",
  "term_label": "mitochondrion",
  "gene_name": "Pyruvate dehydrogenase phosphatase regulatory subunit, mitochondrial"
}